{
  "term_id": "UNKNOWN:0001",
  "gene": "UniProtKB:Q9BSU1",
  "gene_name": "Phagosome assembly factor 1",
  "term_label": "Unknown molecular function",
  "gene_symbol": "PHAF1"
}